regulation of egg-laying behavior [GO:0046662] (biological process) Relationships: is a type of regulation of behavior [GO:0050795]; is a type of regulation of reproductive process [GO:2000241]; regulates egg-laying behavior [GO:0018991] Also known as: regulation of oviposition, regulation of post-mating oviposition Definition: Any process that modulates the frequency, rate or extent of the deposition of eggs, either fertilized or not, upon a surface or into a medium. References: PMID:11932766 Sources: GOC:dph, GOC:tb Subtypes: GO:1901045, positive regulation of egg-laying behavior [GO:1901046]